regulation of lipid transport across blood-brain barrier [GO:1903000] (biological process) Relationships: is a type of GO:0032368; is a type of regulation of transport across blood-brain barrier [GO:0150200]; regulates lipid transport across blood-brain barrier [GO:1990379] Subtypes: negative regulation of lipid transport across blood-brain barrier [GO:1903001], positive regulation of lipid transport across blood-brain barrier [GO:1903002] Also known as: regulation of lipid transport across blood brain barrier References: PMID:24345162 Sources: GOC:TermGenie, GOC:sjp, GO_REF:0000058 Definition: Any process that modulates the frequency, rate or extent of lipid transport across blood-brain barrier.